reticulophagy [GO:0061709] (BP) Definition: The selective autohagy process in which parts of the endoplasmic reticulum are loaded into autophagosomes, delivered to the vacuole, and degraded in response to changing cellular conditions. Relationships: is a type of macroautophagy [GO:0016236] Also known as: ER autophagy, ER-phagy, autophagy of the ER, autophagy of the endoplasmic reticulum, endoplasmic reticulum autophagy, ER degradation, endoplasmic reticulum degradation Regulation: regulated by regulation of reticulophagy [GO:0140500]; positively regulated by GO:0140501 References: PMID:22481944, PMID:24060720, PMID:26040717 Sources: GOC:autophagy, GOC:dph